{
  "gene_name": "Ribosomal protein S6 kinase alpha-1",
  "term_id": "GO:0005737",
  "gene_symbol": "RPS6KA1",
  "term_label": "cytoplasm",
  "gene": "UniProtKB:Q15418"
}